{
  "gene": "UniProtKB:A0A0C4DH63",
  "term_id": "UNKNOWN:0003",
  "gene_symbol": "TRGJP",
  "term_label": "Unknown cellular component",
  "gene_name": "T cell receptor gamma joining P (Fragment)"
}